regulation of cellular response to insulin stimulus [GO:1900076] (biological process) Relationships: is a type of regulation of response to stimulus [GO:0048583]; is a type of GO:0050794; regulates GO:0032869 Subtypes: negative regulation of cellular response to insulin stimulus [GO:1900077], positive regulation of cellular response to insulin stimulus [GO:1900078] Definition: Any process that modulates the frequency, rate or extent of cellular response to insulin stimulus. Sources: GOC:TermGenie, GOC:yaf